L-glutamine:pyruvate aminotransferase activity [GO:0047945] (molecular function) Relationships: is_a L-glutamine aminotransferase activity [GO:0070548] Definition: Catalysis of the reaction: L-glutamine + pyruvate = 2-oxoglutaramate + L-alanine. Also known as: glutamine transaminase L activity, glutamine transaminase activity, glutamine--oxo-acid transaminase activity, glutamine--pyruvate aminotransferase activity, glutamine-alpha-keto acid transamidase activity, glutamine-alpha-keto acid transaminase activity, glutamine-keto acid aminotransferase activity, glutamine-oxo acid aminotransferase activity, glutamine-pyruvate transaminase activity, L-glutamine transaminase L, gamma-glutaminyltransferase activity, glutaminase II activity Sources: EC:2.6.1.15, RHEA:10400